{
  "term_label": "cytoplasm",
  "gene": "UniProtKB:Q9BZX4",
  "gene_name": "Ropporin-1B",
  "term_id": "GO:0005737",
  "gene_symbol": "ROPN1B"
}